SA node cell to atrial cardiac muscle cell signaling [GO:0086018] (biological process) Also known as: SA node cardiac muscle cell to atrial cardiac muscle cell signalling, SA node cardiomyocyte to atrial cardiomyocyte signalling, SAN cardiomyocyte to atrial cardiomyocyte signalling, sinoatrial node cardiomyocyte to atrial cardiomyocyte signalling, sinus node cardiomyocyte to atrial cardiomyocyte signalling Sources: GOC:BHF, GOC:mtg_cardiac_conduct_nov11 Definition: Any process that mediates the transfer of information from an SA node cardiomyocyte to an atrial cardiomyocyte. Relationships: is a type of cell-cell signaling involved in cardiac conduction [GO:0086019]; is a type of GO:0086070